{
  "term_id": "GO:0030317",
  "gene_name": "Protamine-3",
  "gene": "UniProtKB:Q9NNZ6",
  "gene_symbol": "PRM3",
  "term_label": "flagellated sperm motility"
}